monodictyphenone metabolic process [GO:1900813] (biological process) Relationships: is a type of GO:0018958; is a type of secondary metabolic process [GO:0019748]; is a type of carboxylic acid metabolic process [GO:0019752]; is a type of ketone metabolic process [GO:0042180]; is a type of benzene-containing compound metabolic process [GO:0042537] Definition: The chemical reactions and pathways involving monodictyphenone. Subtypes: monodictyphenone catabolic process [GO:1900814], monodictyphenone biosynthetic process [GO:1900815] Sources: GOC:TermGenie, GOC:di Also known as: monodictyphenone metabolism